{
  "gene_symbol": "LARS2",
  "gene": "UniProtKB:Q15031",
  "term_id": "GO:0032543",
  "term_label": "mitochondrial translation",
  "gene_name": "Leucine--tRNA ligase, mitochondrial"
}